{
  "gene_name": "Angiogenin",
  "gene": "UniProtKB:P03950",
  "term_id": "GO:0061844",
  "gene_symbol": "ANG",
  "term_label": "antimicrobial humoral immune response mediated by antimicrobial peptide"
}